{
  "gene_symbol": "COA6",
  "gene_name": "Cytochrome c oxidase assembly factor 6 homolog",
  "term_id": "UNKNOWN:0001",
  "gene": "UniProtKB:Q5JTJ3",
  "term_label": "Unknown molecular function"
}